{
  "gene": "UniProtKB:Q9NPI0",
  "gene_name": "Transmembrane protein 138",
  "term_label": "Unknown biological process",
  "gene_symbol": "TMEM138",
  "term_id": "UNKNOWN:0002"
}